{
  "term_id": "GO:0043015",
  "term_label": "gamma-tubulin binding",
  "gene_symbol": "TUBGCP4",
  "gene_name": "Gamma-tubulin complex component 4",
  "gene": "UniProtKB:Q9UGJ1"
}